{
  "gene_name": "Sodium-dependent organic anion transporter",
  "term_id": "GO:0015721",
  "gene": "UniProtKB:Q3KNW5",
  "term_label": "bile acid and bile salt transport",
  "gene_symbol": "SLC10A6"
}